{
  "gene": "UniProtKB:Q5HYJ3",
  "gene_symbol": "FAM76B",
  "gene_name": "Protein FAM76B",
  "term_label": "nuclear speck",
  "term_id": "GO:0016607"
}